{
  "gene_symbol": "MRPL32",
  "term_label": "structural constituent of ribosome",
  "gene_name": "Large ribosomal subunit protein bL32m",
  "term_id": "GO:0003735",
  "gene": "UniProtKB:Q9BYC8"
}